{
  "gene_symbol": "SLC22A15",
  "gene_name": "Solute carrier family 22 member 15",
  "gene": "UniProtKB:Q8IZD6",
  "term_id": "UNKNOWN:0002",
  "term_label": "Unknown biological process"
}